positive regulation of protein polyglycylation [GO:1903346] (biological process) Relationships: is a type of positive regulation of protein modification process [GO:0031401]; is a type of regulation of protein polyglycylation [GO:1903344]; positively regulates protein polyglycylation [GO:0018094] Definition: Any process that activates or increases the frequency, rate or extent of protein polyglycylation. References: PMID:21298005 Sources: GOC:TermGenie, GOC:sart, GO_REF:0000058 Also known as: up regulation of protein polyglycylation, up-regulation of protein polyglycylation, upregulation of protein polyglycylation, activation of protein polyglycylation